{
  "gene_name": "Tyrosine-protein kinase Yes",
  "gene": "UniProtKB:P07947",
  "term_label": "cell differentiation",
  "gene_symbol": "YES1",
  "term_id": "GO:0030154"
}